{
  "term_id": "GO:0019841",
  "term_label": "retinol binding",
  "gene_name": "Retinol-binding protein 4",
  "gene_symbol": "RBP4",
  "gene": "UniProtKB:P02753"
}